release from viral latency [GO:0019046] (biological process) Relationships: is a type of viral process [GO:0016032]; is part of latent virus replication [GO:0019045] Subtypes: provirus excision [GO:0032359] Sources: GOC:dos, GOC:jl Regulation: RO_0002211 by latency-replication decision [GO:0098689] Definition: The process by which a virus begins to replicate following a latency replication decision (switch).